{
  "gene_name": "G-protein coupled receptor 171",
  "term_label": "G protein-coupled receptor signaling pathway",
  "gene": "UniProtKB:O14626",
  "gene_symbol": "GPR171",
  "term_id": "GO:0007186"
}